{
  "gene": "UniProtKB:P31273",
  "term_label": "RNA polymerase II transcription regulatory region sequence-specific DNA binding",
  "gene_name": "Homeobox protein Hox-C8",
  "term_id": "GO:0000977",
  "gene_symbol": "HOXC8"
}